very-low-density lipoprotein particle receptor activity [GO:0030229] (molecular function) Also known as: VLDL receptor, very-low-density lipoprotein receptor activity, apolipoprotein E receptor activity Sources: GOC:bf, ISBN:0198506732 Relationships: is a type of lipoprotein particle receptor activity [GO:0030228]; has part very-low-density lipoprotein particle binding [GO:0034189] Definition: Combining with a very-low-density lipoprotein particle and delivering the very-low-density lipoprotein into the cell via endocytosis.